galactokinase activity [GO:0004335] (molecular function) Also known as: ATP:D-galactose 1-phosphotransferase activity, ATP:D-galactose-1-phosphotransferase activity, galactokinase (phosphorylating) Relationships: is a type of phosphotransferase activity, alcohol group as acceptor [GO:0016773]; is a type of GO:0019200 Sources: EC:2.7.1.6, RHEA:13553 Definition: Catalysis of the reaction: D-galactose + ATP = alpha-D-galactose 1-phosphate + ADP + 2 H+.